{
  "gene_name": "Cathepsin W",
  "gene_symbol": "CTSW",
  "gene": "UniProtKB:P56202",
  "term_label": "lysosome",
  "term_id": "GO:0005764"
}